homoisocitrate dehydrogenase activity [GO:0047046] (molecular function) Definition: Catalysis of the reaction: NAD+ + 3-carboxy-2-hydroxyadipate = NADH + H+ + CO2 + 2-keto-adipate. Note: Note that EC:1.1.1.155 was merged into EC:1.1.1.87 as they are identical. Relationships: is a type of oxidoreductase activity, acting on the CH-OH group of donors, NAD or NADP as acceptor [GO:0016616] Sources: EC:1.1.1.87 Also known as: 3-carboxy-2-hydroxyadipate dehydrogenase activity, (-)-1-hydroxy-1,2,4-butanetricarboxylate:NAD(+) oxidoreductase (decarboxylating) activity, (-)-1-hydroxy-1,2,4-butanetricarboxylate:NAD+ oxidoreductase (decarboxylating), (1R,2S)-1-hydroxybutane-1,2,4-tricarboxylate:NAD+ oxidoreductase (decarboxylating), 2-hydroxy-3-carboxyadipate dehydrogenase activity, 3-carboxy-2-hydroxyadipate:NAD(+) oxidoreductase (decarboxylating) activity, 3-carboxy-2-hydroxyadipate:NAD+ oxidoreductase (decarboxylating), homoisocitric dehydrogenase activity